{
  "gene_symbol": "RPL37AP8",
  "gene_name": "Putative ribosomal protein eL43-like",
  "term_label": "Unknown molecular function",
  "gene": "UniProtKB:A6NKH3",
  "term_id": "UNKNOWN:0001"
}